{
  "gene_name": "GTPase-activating protein and VPS9 domain-containing protein 1",
  "gene_symbol": "GAPVD1",
  "gene": "UniProtKB:Q14C86",
  "term_id": "GO:0005829",
  "term_label": "cytosol"
}